{
  "term_label": "central nervous system development",
  "gene_name": "Neurocan core protein",
  "gene_symbol": "NCAN",
  "term_id": "GO:0007417",
  "gene": "UniProtKB:O14594"
}